guanine phosphoribosyltransferase activity [GO:0052657] (molecular function) Relationships: is a type of purine phosphoribosyltransferase activity [GO:0106130] Sources: RHEA:25424 Also known as: Transphosphoribosidase activity, guanine-hypoxanthine phosphoribosyltransferase activity, hypoxanthine-guanine phosphoribosyltransferase activity, 6-hydroxypurine phosphoribosyltransferase activity, 6-mercaptopurine phosphoribosyltransferase activity, GMP pyrophosphorylase activity, GPRT, guanosine 5'-phosphate pyrophosphorylase activity, guanosine phosphoribosyltransferase activity, guanylate pyrophosphorylase activity, guanylic pyrophosphorylase activity, purine-6-thiol phosphoribosyltransferase activity Definition: Catalysis of the reaction: GMP + diphosphate = guanine + 5-phospho-alpha-D-ribose 1-diphosphate.